{
  "gene_name": "Uncharacterized protein C11orf21",
  "term_id": "UNKNOWN:0001",
  "gene": "UniProtKB:Q9P2W6",
  "gene_symbol": "C11orf21",
  "term_label": "Unknown molecular function"
}